{
  "term_label": "postsynaptic density membrane",
  "gene_symbol": "NETO1",
  "gene_name": "Neuropilin and tolloid-like protein 1",
  "gene": "UniProtKB:Q8TDF5",
  "term_id": "GO:0098839"
}